tetrahydroxynaphthalene reductase activity [GO:0047039] (molecular function) Sources: EC:1.1.1.252, MetaCyc:1.1.1.252-RXN Also known as: T4HN reductase activity, scytalone:NADP+ delta5-oxidoreductase activity Definition: Catalysis of the reaction: NADP+ + scytalone = NADPH + H+ + 1,3,6,8-naphthalenetetrol. Relationships: is a type of oxidoreductase activity, acting on the CH-OH group of donors, NAD or NADP as acceptor [GO:0016616]